{
  "gene_symbol": "IFIT2",
  "gene": "UniProtKB:P09913",
  "term_label": "RNA binding",
  "gene_name": "Interferon-induced protein with tetratricopeptide repeats 2",
  "term_id": "GO:0003723"
}